{
  "term_label": "cytoplasm",
  "gene": "UniProtKB:Q99569",
  "gene_symbol": "PKP4",
  "gene_name": "Plakophilin-4",
  "term_id": "GO:0005737"
}